establishment of plastid localization [GO:0051667] (biological process) Also known as: establishment of plastid localisation Subtypes: chloroplast relocation [GO:0009902] Relationships: is a type of plastid localization [GO:0051644]; is_a establishment of localization in cell [GO:0051649]; is a type of establishment of organelle localization [GO:0051656] Sources: GOC:ai Definition: The directed movement of a plastid to a specific location in the cell.